{
  "term_label": "mRNA splicing, via spliceosome",
  "term_id": "GO:0000398",
  "gene_symbol": "SNRPA",
  "gene_name": "U1 small nuclear ribonucleoprotein A",
  "gene": "UniProtKB:P09012"
}